{
  "term_id": "GO:0030867",
  "gene": "UniProtKB:Q8N5G2",
  "term_label": "rough endoplasmic reticulum membrane",
  "gene_name": "Macoilin",
  "gene_symbol": "MACO1"
}